{
  "term_label": "plasma membrane",
  "gene_symbol": "SLC1A4",
  "gene": "UniProtKB:P43007",
  "gene_name": "Neutral amino acid transporter A",
  "term_id": "GO:0005886"
}